{
  "term_label": "NADP binding",
  "gene": "UniProtKB:Q13423",
  "gene_symbol": "NNT",
  "gene_name": "NAD(P) transhydrogenase, mitochondrial",
  "term_id": "GO:0050661"
}